{
  "term_label": "nucleus",
  "gene": "UniProtKB:Q4V348",
  "gene_symbol": "ZNF658B",
  "term_id": "GO:0005634",
  "gene_name": "Zinc finger protein 658B"
}